{
  "term_label": "cytoplasm",
  "gene_symbol": "PER2",
  "term_id": "GO:0005737",
  "gene_name": "Period circadian protein homolog 2",
  "gene": "UniProtKB:O15055"
}